4-hydroxyphenylacetate decarboxylase activity [GO:0043722] (molecular function) Definition: Catalysis of the reaction: (4-hydroxyphenyl)acetate + H+ = 4-cresol + CO2. Sources: EC:4.1.1.83, RHEA:22732 Also known as: 4-(hydroxyphenyl)acetate carboxy-lyase (4-methylphenol-forming), 4-Hpd activity, 4-hydroxyphenylacetate carboxy-lyase activity, p-Hpd activity, p-hydroxyphenylacetate decarboxylase activity Relationships: is a type of carboxy-lyase activity [GO:0016831]